{
  "term_label": "morphogenesis of an epithelium",
  "gene": "UniProtKB:A0A140TA62",
  "gene_symbol": "LOC100653049",
  "term_id": "GO:0002009",
  "gene_name": "IF rod domain-containing protein"
}